{
  "term_id": "GO:0005111",
  "gene_symbol": "FGF8",
  "gene_name": "Fibroblast growth factor 8",
  "gene": "UniProtKB:P55075",
  "term_label": "type 2 fibroblast growth factor receptor binding"
}